{
  "term_label": "nucleus",
  "term_id": "GO:0005634",
  "gene_name": "Rhox homeobox family member 2",
  "gene": "UniProtKB:Q9BQY4",
  "gene_symbol": "RHOXF2"
}